{
  "term_label": "extracellular space",
  "gene": "UniProtKB:P07477",
  "gene_symbol": "PRSS1",
  "term_id": "GO:0005615",
  "gene_name": "Serine protease 1"
}